{
  "term_id": "GO:0034451",
  "gene_symbol": "CCDC57",
  "gene_name": "Coiled-coil domain-containing protein 57",
  "gene": "UniProtKB:Q2TAC2",
  "term_label": "centriolar satellite"
}